{
  "term_label": "cytoplasm",
  "gene_symbol": "LRRD1",
  "gene_name": "Leucine-rich repeat and death domain-containing protein 1",
  "term_id": "GO:0005737",
  "gene": "UniProtKB:A4D1F6"
}